{
  "gene_name": "Serine_threonine-protein kinase_endoribonuclease IRE2",
  "gene_symbol": "ERN2",
  "term_id": "GO:0070059",
  "gene": "UniProtKB:Q76MJ5",
  "term_label": "intrinsic apoptotic signaling pathway in response to endoplasmic reticulum stress"
}